microtubule-based protein transport [GO:0099118] (BP) Definition: A microtubule-based process that results in the transport of proteins. Sources: GOC:vw Relationships: is a type of protein transport [GO:0015031]; is a type of microtubule-based transport [GO:0099111] Subtypes: protein transport along microtubule [GO:0098840], microtubule polymerization based protein transport [GO:0099112]